putrescine transport [GO:0015847] (biological process) Relationships: is a type of GO:0015695; is a type of GO:0015846 Sources: GOC:krc, ISBN:0198506732 Definition: The directed movement of putrescine into, out of or within a cell, or between cells, by means of some agent such as a transporter or pore. Putrescine is 1,4-diaminobutane, the polyamine formed by decarboxylation of ornithine and the metabolic precursor of spermidine and spermine.